{
  "gene_symbol": "DDX17",
  "term_id": "GO:0005737",
  "term_label": "cytoplasm",
  "gene_name": "Probable ATP-dependent RNA helicase DDX17",
  "gene": "UniProtKB:Q92841"
}